{
  "gene_symbol": "HLA-DPA1",
  "gene_name": "HLA class II histocompatibility antigen, DP alpha 1 chain",
  "term_id": "GO:0019886",
  "term_label": "antigen processing and presentation of exogenous peptide antigen via MHC class II",
  "gene": "UniProtKB:P20036"
}